RNA-templated transcription [GO:0001172] (BP) Definition: The synthesis of an RNA transcript from an RNA template. Sources: GOC:txnOH Subtypes: GO:0140745 Also known as: transcription, RNA-dependent, transcription, RNA-templated Relationships: is a type of RNA biosynthetic process [GO:0032774]; is part of gene expression [GO:0010467]